nuclear pore transmembrane ring [GO:0070762] (cellular component) Relationships: is_a nuclear protein-containing complex [GO:0140513]; is part of nuclear pore [GO:0005643] Also known as: NDC1 complex, NDC1 subcomplex References: PMID:18046406, PMID:19524430, PMID:20947011, PMID:22419078 Sources: GOC:dgf Definition: A subcomplex of the nuclear pore complex (NPC) that spans the nuclear membrane and anchors the NPC to the nuclear envelope. In S. cerevisiae, the transmembrane ring is composed of Pom152p, Pom34p, and Ndc1p. In vertebrates, it is composed of Gp210, Ndc1, and Pom121. Components are arranged in 8-fold symmetrical 'spokes' around the central transport channel. A single 'spoke', can be isolated and is sometime referred to as the Ndc1 complex.